{
  "gene": "UniProtKB:Q6ZN92",
  "term_label": "dUTP diphosphatase activity",
  "gene_name": "Putative inactive deoxyuridine 5'-triphosphate nucleotidohydrolase-like protein FLJ16323",
  "gene_symbol": "Q6ZN92",
  "term_id": "GO:0004170"
}